{
  "gene_symbol": "PRF1",
  "gene": "UniProtKB:P14222",
  "term_id": "GO:0016020",
  "term_label": "membrane",
  "gene_name": "Perforin-1"
}